thyrotropin-releasing hormone receptor activity [GO:0004997] (molecular function) Relationships: is a type of G protein-coupled receptor activity [GO:0004930] Definition: Combining with thyrotropin-releasing hormone to initiate a change in cell activity. Sources: GOC:mah